{
  "gene_name": "5-aminolevulinate synthase, erythroid-specific, mitochondrial",
  "term_id": "GO:0005739",
  "term_label": "mitochondrion",
  "gene": "UniProtKB:P22557",
  "gene_symbol": "ALAS2"
}